hypochlorous acid biosynthetic process [GO:0002149] (biological process) Also known as: HClO biosynthetic process, HOCl biosynthetic process, hypochlorous acid biosynthesis, hypochlorite biosynthetic process Definition: The chemical reactions and pathways resulting in the formation of hypochlorous acid. Note: Note that this reaction is catalyzed by myeloperoxidase in neutrophils. Relationships: is a type of oxoacid metabolic process [GO:0043436]; is a type of small molecule biosynthetic process [GO:0044283]; is a type of GO:1903409 References: PMID:10085024, PMID:176150 Sources: GOC:add